{
  "term_id": "GO:0036158",
  "gene_name": "Coiled-coil domain-containing protein 63",
  "term_label": "outer dynein arm assembly",
  "gene_symbol": "CCDC63",
  "gene": "UniProtKB:Q8NA47"
}